mannosyltransferase activity [GO:0000030] (molecular function) Subtypes: alpha-1,6-mannosyltransferase activity [GO:0000009], alpha-1,2-mannosyltransferase activity [GO:0000026], GO:0000033, dolichyl-phosphate-mannose-protein mannosyltransferase activity [GO:0004169], GPI mannosyltransferase activity [GO:0004376], dolichyl-phosphate beta-D-mannosyltransferase activity [GO:0004582], GO:0016438, beta-1,4-mannosyltransferase activity [GO:0019187], GO:0047252, GO:0047264, undecaprenyl-phosphate mannosyltransferase activity [GO:0047267], alpha-1,4-mannosyltransferase activity [GO:0051751], GO:0103064, GO:0120562 Definition: Catalysis of the transfer of a mannosyl group to an acceptor molecule, typically another carbohydrate or a lipid. Relationships: is a type of hexosyltransferase activity [GO:0016758] Sources: GOC:ai, GOC:cjm